positive regulation of establishment of competence for transformation [GO:0045809] (biological process) Relationships: is a type of regulation of establishment of competence for transformation [GO:0045304]; is a type of positive regulation of cellular process [GO:0048522]; is a type of positive regulation of response to stimulus [GO:0048584]; positively regulates GO:0030420 Also known as: up regulation of establishment of competence for transformation, up-regulation of establishment of competence for transformation, upregulation of establishment of competence for transformation, activation of establishment of competence for transformation, stimulation of establishment of competence for transformation, activator of the establishment of competence for transformation activity Sources: GOC:go_curators Definition: Any process that activates or increases the frequency, rate or extent of establishment of competence for transformation.